{
  "gene_symbol": "TSC22D1",
  "gene": "UniProtKB:Q15714",
  "gene_name": "TSC22 domain family protein 1",
  "term_id": "UNKNOWN:0001",
  "term_label": "Unknown molecular function"
}